{
  "gene_name": "Cellular communication network factor 6",
  "gene_symbol": "CCN6",
  "term_id": "GO:0008201",
  "gene": "UniProtKB:O95389",
  "term_label": "heparin binding"
}